{
  "term_label": "Unknown biological process",
  "gene": "UniProtKB:Q8N8A6",
  "gene_name": "ATP-dependent RNA helicase DDX51",
  "gene_symbol": "DDX51",
  "term_id": "UNKNOWN:0002"
}